{
  "gene_symbol": "SYTL4",
  "term_id": "GO:0042043",
  "gene": "UniProtKB:Q96C24",
  "gene_name": "Synaptotagmin-like protein 4",
  "term_label": "neurexin family protein binding"
}